{
  "term_label": "L-tryptophan catabolic process to acetyl-CoA",
  "term_id": "GO:0019442",
  "gene_name": "Tryptophan 2,3-dioxygenase",
  "gene": "UniProtKB:P48775",
  "gene_symbol": "TDO2"
}